vitamin D biosynthetic process [GO:0042368] (biological process) Subtypes: GO:0036378, GO:1901755 Relationships: is a type of steroid biosynthetic process [GO:0006694]; is a type of vitamin D metabolic process [GO:0042359]; is a type of GO:0042362 Also known as: vitamin D anabolism, vitamin D biosynthesis, vitamin D formation, vitamin D synthesis, calciferol biosynthesis, calciferol biosynthetic process, cholecalciferol biosynthesis, cholecalciferol biosynthetic process, ergocalciferol biosynthesis, ergocalciferol biosynthetic process Definition: The chemical reactions and pathways resulting in the formation of vitamin D, any of a group of related, fat-soluble compounds that are derived from delta-5,7 steroids and play a central role in calcium metabolism. Specific forms of vitamin D include calciferol (ergocalciferol; vitamin D2) and cholecalciferol (calciol; vitamin D3). Regulation: negatively regulated by negative regulation of vitamin D biosynthetic process [GO:0010957]; regulated by regulation of vitamin D biosynthetic process [GO:0060556]; positively regulated by positive regulation of vitamin D biosynthetic process [GO:0060557] Sources: GOC:mah, ISBN:0471331309